{
  "gene_symbol": "SEMA3A",
  "gene_name": "Semaphorin-3A",
  "gene": "UniProtKB:Q14563",
  "term_id": "GO:0005615",
  "term_label": "extracellular space"
}